{
  "gene_name": "Immunoglobulin lambda variable 2-23",
  "term_id": "GO:0006955",
  "term_label": "immune response",
  "gene": "UniProtKB:P01705",
  "gene_symbol": "IGLV2-23"
}